floral organ development [GO:0048437] (biological process) Relationships: is_a developmental process involved in reproduction [GO:0003006]; is a type of plant organ development [GO:0099402]; is part of flower development [GO:0009908] Sources: GOC:PO_curators, GOC:go_curators, PO:0025395 Definition: The process whose specific outcome is the progression of the floral organ over time, from its formation to the mature structure. Subtypes: carpel development [GO:0048440], petal development [GO:0048441], sepal development [GO:0048442], stamen development [GO:0048443]